glycerol transmembrane transporter activity [GO:0015168] (molecular function) Subtypes: glycerol channel activity [GO:0015254] Definition: Enables the transfer of glycerol from one side of a membrane to the other. Glycerol is 1,2,3-propanetriol, a sweet, hygroscopic, viscous liquid, widely distributed in nature as a constituent of many lipids. Sources: GOC:ai Relationships: is a type of GO:0015144; is a type of polyol transmembrane transporter activity [GO:0015166]; is part of glycerol transmembrane transport [GO:0015793]